{
  "gene_name": "Histone H2B type 1-H",
  "term_id": "GO:0000786",
  "gene": "UniProtKB:Q93079",
  "term_label": "nucleosome",
  "gene_symbol": "H2BC9"
}